host cell endomembrane system [GO:0033645] (cellular component) Definition: A collection of membranous structures involved in transport within the host cell. The main components of the endomembrane system are endoplasmic reticulum, Golgi bodies, vesicles, cell membrane and nuclear envelope. Members of the endomembrane system pass materials through each other or though the use of vesicles. The host is defined as the larger of the organisms involved in a symbiotic interaction. Sources: GOC:pamgo_curators Relationships: is a type of host cell membrane [GO:0033644]